{
  "gene_name": "Olfactory receptor 5H1",
  "gene": "UniProtKB:A6NKK0",
  "term_label": "odorant binding",
  "term_id": "GO:0005549",
  "gene_symbol": "OR5H1"
}